{
  "term_label": "astrocyte activation",
  "term_id": "GO:0048143",
  "gene_symbol": "CNTF",
  "gene": "UniProtKB:P26441",
  "gene_name": "Ciliary neurotrophic factor"
}